{
  "term_id": "GO:0010754",
  "gene": "UniProtKB:Q9Y233",
  "gene_symbol": "PDE10A",
  "term_label": "negative regulation of receptor guanylyl cyclase signaling pathway",
  "gene_name": "cAMP and cAMP-inhibited cGMP 3',5'-cyclic phosphodiesterase 10A"
}